modulation of nutrient release by host [GO:0052091] (biological process) Also known as: modulation by symbiont of nutrient release from host Subtypes: positive regulation of nutrient release by host [GO:0052092] Definition: Any process in which an organism modulates the frequency, rate or extent of the release of nutrients from its host organism. The host is defined as the larger of the organisms involved in a symbiotic interaction. Relationships: is a type of acquisition of nutrients from host [GO:0044002] Sources: GOC:mtg_pamgo_17jul06